{
  "term_label": "cytosolic large ribosomal subunit",
  "gene": "UniProtKB:P42766",
  "gene_symbol": "RPL35",
  "gene_name": "Large ribosomal subunit protein uL29",
  "term_id": "GO:0022625"
}